{
  "gene_symbol": "SSRP1",
  "term_id": "GO:1902275",
  "term_label": "regulation of chromatin organization",
  "gene": "UniProtKB:Q08945",
  "gene_name": "FACT complex subunit SSRP1"
}